Rho protein signal transduction [GO:0007266] (biological process) Definition: An intracellular signaling cassette in which a small monomeric GTPase of the Rho subfamily relays a signal. Sources: GOC:bf Also known as: Rho mediated signal transduction Relationships: is a type of small GTPase-mediated signal transduction [GO:0007264] Subtypes: GO:0032488 Regulation: RO_0002211 by regulation of Rho protein signal transduction [GO:0035023]; negatively regulated by negative regulation of Rho protein signal transduction [GO:0035024]; positively regulated by positive regulation of Rho protein signal transduction [GO:0035025]